{
  "gene": "UniProtKB:Q8NI27",
  "term_id": "GO:0000445",
  "gene_symbol": "THOC2",
  "term_label": "THO complex part of transcription export complex",
  "gene_name": "THO complex subunit 2"
}